{
  "gene_name": "Actin-related protein T2",
  "term_id": "GO:0005200",
  "gene_symbol": "ACTRT2",
  "term_label": "structural constituent of cytoskeleton",
  "gene": "UniProtKB:Q8TDY3"
}